synoviocyte proliferation [GO:0002941] (biological process) References: PMID:10770586, PMID:9546370 Regulation: regulated by regulation of synoviocyte proliferation [GO:1901645]; negatively regulated by negative regulation of synoviocyte proliferation [GO:1901646]; positively regulated by positive regulation of synoviocyte proliferation [GO:1901647] Definition: The multiplication or reproduction of type B synoviocytes by cell division, resulting in the expansion of their population. A type B synoviocyte is a fibroblast-like cell found in synovial tissues. Relationships: is a type of GO:0050673